positive regulation of cellotriose transport [GO:1900287] (biological process) Also known as: up regulation of cellotriose transport, up-regulation of cellotriose transport, upregulation of cellotriose transport, activation of cellotriose transport Relationships: is a type of positive regulation of transport [GO:0051050]; is a type of regulation of cellotriose transport [GO:1900285]; positively regulates cellotriose transport [GO:2001096] Sources: GOC:TermGenie, GOC:mengo_curators Definition: Any process that activates or increases the frequency, rate or extent of cellotriose transport.